{
  "gene_symbol": "PRSS57",
  "term_id": "GO:0051604",
  "gene": "UniProtKB:Q6UWY2",
  "gene_name": "Serine protease 57",
  "term_label": "protein maturation"
}